{
  "term_id": "UNKNOWN:0003",
  "gene_name": "Uncharacterized protein",
  "term_label": "Unknown cellular component",
  "gene": "UniProtKB:A0A804HI29",
  "gene_symbol": "A0A804HI29"
}